{
  "term_id": "UNKNOWN:0001",
  "gene": "UniProtKB:Q9Y3T6",
  "gene_symbol": "R3HCC1",
  "term_label": "Unknown molecular function",
  "gene_name": "R3H and coiled-coil domain-containing protein 1"
}